UFM1 conjugating enzyme activity [GO:0061657] (molecular function) Relationships: is a type of ubiquitin-like protein conjugating enzyme activity [GO:0061650]; is a type of GO:0071568 Also known as: E2 Sources: GOC:dph Definition: Isoenergetic transfer of UFM1 from one protein to another via the reaction X-UFM1 + Y = Y-UFM1 + X, where both the X-UFM1 and Y-UFM1 linkages are thioester bonds between the C-terminal amino acid of UFM1 and a sulfhydryl side group of a cysteine residue.